{
  "gene_symbol": "FOXI2",
  "gene": "UniProtKB:Q6ZQN5",
  "gene_name": "Forkhead box protein I2",
  "term_id": "GO:0009653",
  "term_label": "anatomical structure morphogenesis"
}